{
  "gene_symbol": "DCPS",
  "term_id": "GO:0000290",
  "gene": "UniProtKB:Q96C86",
  "term_label": "deadenylation-dependent decapping of nuclear-transcribed mRNA",
  "gene_name": "m7GpppX diphosphatase"
}